chlororespiration [GO:0010478] (biological process) Relationships: is a type of GO:0022904 Definition: A respiratory electron flow (from NAD(P)H to plastoquinone (PQ) and O2) involving both a nonphotochemical reduction and re-oxidation of PQ pool. References: PMID:17573537 Sources: GOC:mtg_electron_transport, GOC:tb